{
  "gene": "UniProtKB:Q8TB33",
  "term_id": "UNKNOWN:0003",
  "term_label": "Unknown cellular component",
  "gene_name": "Putative uncharacterized protein encoded by LINC01560",
  "gene_symbol": "LINC01560"
}